{
  "term_label": "protein ubiquitination",
  "gene": "UniProtKB:P0CG47",
  "gene_name": "Polyubiquitin-B",
  "term_id": "GO:0016567",
  "gene_symbol": "UBB"
}